{
  "gene_name": "Mitochondrial import receptor subunit TOM7 homolog",
  "term_id": "UNKNOWN:0001",
  "term_label": "Unknown molecular function",
  "gene": "UniProtKB:Q9P0U1",
  "gene_symbol": "TOMM7"
}